{
  "gene_symbol": "RAB3C",
  "gene_name": "Ras-related protein Rab-3C",
  "term_label": "exocytosis",
  "term_id": "GO:0006887",
  "gene": "UniProtKB:Q96E17"
}